contractile vacuole localization [GO:0140027] (biological process) Relationships: is_a vesicle localization [GO:0051648]; is a type of vacuolar localization [GO:1990849] References: PMID:19687255 Also known as: establishment of contractile vacuole localization Definition: The directed movement of the contractile vacuole to a specific location.